{
  "gene_symbol": "ANKFY1",
  "term_id": "GO:0042147",
  "gene": "UniProtKB:Q9P2R3",
  "gene_name": "Rabankyrin-5",
  "term_label": "retrograde transport, endosome to Golgi"
}